{
  "gene_symbol": "OIT3",
  "gene_name": "Oncoprotein-induced transcript 3 protein",
  "term_label": "Unknown biological process",
  "gene": "UniProtKB:Q8WWZ8",
  "term_id": "UNKNOWN:0002"
}